{
  "gene_symbol": "AVPR1B",
  "gene": "UniProtKB:P47901",
  "term_id": "GO:0005886",
  "term_label": "plasma membrane",
  "gene_name": "Vasopressin V1b receptor"
}